{
  "gene_symbol": "CHRNB3",
  "term_id": "GO:0095500",
  "gene_name": "Neuronal acetylcholine receptor subunit beta-3",
  "gene": "UniProtKB:Q05901",
  "term_label": "acetylcholine receptor signaling pathway"
}